{
  "term_id": "UNKNOWN:0002",
  "term_label": "Unknown biological process",
  "gene_symbol": "LRFN3",
  "gene": "UniProtKB:Q9BTN0",
  "gene_name": "Leucine-rich repeat and fibronectin type-III domain-containing protein 3"
}